L-dopa decarboxylase activity [GO:0036468] (molecular function) Sources: GOC:PARL, GOC:bf, RHEA:12272 Relationships: is a type of aromatic-L-amino-acid decarboxylase activity [GO:0004058] Regulation: positively regulated by GO:0036478 Definition: Catalysis of the reaction: L-dopa + H+ = CO2 + dopamine. Also known as: 4-dihydroxyl-L-phenylalanine decarboxylase activity, DDC activity, DOPA decarboxylase activity